{
  "gene_name": "Calcium uniporter regulatory subunit MCUb, mitochondrial",
  "gene": "UniProtKB:Q9NWR8",
  "gene_symbol": "MCUB",
  "term_id": "GO:0036444",
  "term_label": "calcium import into the mitochondrion"
}